regulation of single-species biofilm formation on inanimate substrate [GO:1900231] (biological process) Definition: Any process that modulates the frequency, rate or extent of single-species biofilm formation on inanimate substrate. Sources: GOC:TermGenie, GOC:di Relationships: is a type of regulation of single-species biofilm formation [GO:1900190]; regulates GO:0044011 Subtypes: negative regulation of single-species biofilm formation on inanimate substrate [GO:1900232], positive regulation of single-species biofilm formation on inanimate substrate [GO:1900233]